{
  "gene_name": "Sodium- and chloride-dependent GABA transporter 1",
  "term_id": "GO:0005886",
  "term_label": "plasma membrane",
  "gene_symbol": "SLC6A1",
  "gene": "UniProtKB:P30531"
}